{
  "gene_symbol": "MAP6",
  "gene_name": "Microtubule-associated protein 6",
  "term_id": "GO:0005874",
  "term_label": "microtubule",
  "gene": "UniProtKB:Q96JE9"
}